{
  "term_label": "GTPase activator activity",
  "gene": "UniProtKB:O76081",
  "term_id": "GO:0005096",
  "gene_name": "Regulator of G-protein signaling 20",
  "gene_symbol": "RGS20"
}